{
  "gene": "UniProtKB:Q9NSC5",
  "term_id": "GO:0005886",
  "gene_symbol": "HOMER3",
  "term_label": "plasma membrane",
  "gene_name": "Homer protein homolog 3"
}